{
  "term_id": "GO:0015908",
  "gene_name": "Myelin P2 protein",
  "gene_symbol": "PMP2",
  "gene": "UniProtKB:P02689",
  "term_label": "fatty acid transport"
}